{
  "term_id": "GO:0001570",
  "gene_name": "Cerebral cavernous malformations 2 protein",
  "gene": "UniProtKB:Q9BSQ5",
  "gene_symbol": "CCM2",
  "term_label": "vasculogenesis"
}